{
  "gene_symbol": "CD83",
  "term_id": "UNKNOWN:0003",
  "gene": "UniProtKB:Q01151",
  "term_label": "Unknown cellular component",
  "gene_name": "CD83 antigen"
}